{
  "term_label": "Unknown molecular function",
  "gene_symbol": "KIAA0513",
  "gene_name": "Uncharacterized protein KIAA0513",
  "gene": "UniProtKB:O60268",
  "term_id": "UNKNOWN:0001"
}